{
  "gene": "UniProtKB:P10809",
  "gene_name": "60 kDa heat shock protein, mitochondrial",
  "gene_symbol": "HSPD1",
  "term_id": "GO:0006457",
  "term_label": "protein folding"
}